{
  "gene_symbol": "RSAD2",
  "gene": "UniProtKB:Q8WXG1",
  "term_id": "GO:0005783",
  "term_label": "endoplasmic reticulum",
  "gene_name": "S-adenosylmethionine-dependent nucleotide dehydratase RSAD2"
}